abieta-7,13-dien-18-ol hydroxylase activity [GO:0036204] (molecular function) Relationships: is a type of GO:0016709 Sources: EC:1.14.14.145 Definition: Catalysis of the reaction: abieta-7,13-dien-18-ol + NADPH + H+ + O2 = abieta-7,13-dien-18-al + NADP+ + 2 H2O. This is a two step reaction. The first step is: abieta-7,13-dien-18-ol + NADPH + H+ + O2 = abieta-7,13-dien-18,18-diol + + NADP+ + H2O. The second step is a spontaneous reaction: abieta-7,13-dien-18,18-diol = abieta-7,13-dien-18-al + H2O.